{
  "gene_symbol": "DDX42",
  "term_id": "GO:0005634",
  "term_label": "nucleus",
  "gene_name": "ATP-dependent RNA helicase DDX42",
  "gene": "UniProtKB:Q86XP3"
}